B cell receptor transport into membrane raft [GO:0032597] (biological process) Subtypes: B cell receptor transport into immunological synapse [GO:0032598] Definition: The directed movement of a B cell receptor into a membrane raft. Relationships: is a type of B cell receptor transport within lipid bilayer [GO:0032595]; is a type of protein transport into membrane raft [GO:0032596] Also known as: B cell receptor translocation into membrane raft, B cell receptor transport into lipid raft, BCR translocation into membrane raft, BCR transport into membrane raft Sources: GOC:mah